{
  "gene_name": "Cytosolic phospholipase A2",
  "gene": "UniProtKB:P47712",
  "term_label": "endoplasmic reticulum",
  "term_id": "GO:0005783",
  "gene_symbol": "PLA2G4A"
}